{
  "term_label": "regulation of long-term synaptic potentiation",
  "gene": "UniProtKB:Q7LC44",
  "term_id": "GO:1900271",
  "gene_name": "Activity-regulated cytoskeleton-associated protein",
  "gene_symbol": "ARC"
}